{
  "gene": "UniProtKB:Q8N6M5",
  "gene_symbol": "ALLC",
  "term_id": "UNKNOWN:0003",
  "term_label": "Unknown cellular component",
  "gene_name": "Probable inactive allantoicase"
}